{
  "term_id": "GO:0031593",
  "gene_name": "Ubiquilin-3",
  "gene": "UniProtKB:Q9H347",
  "term_label": "polyubiquitin modification-dependent protein binding",
  "gene_symbol": "UBQLN3"
}